ent-pimara-8(14),15-diene synthase activity [GO:0034282] (molecular function) Sources: RHEA:25540 Definition: Catalysis of the reaction: ent-copalyl diphosphate = ent-pimara-8(14),15-diene + diphosphate. Also known as: ent-pimaradiene synthase activity, ent-copalyl-diphosphate diphosphate-lyase [ent-pimara-8(14),15-diene-forming] activity Relationships: is a type of carbon-oxygen lyase activity, acting on phosphates [GO:0016838]